{
  "term_label": "inflammatory response",
  "gene": "UniProtKB:Q8TAD2",
  "gene_symbol": "IL17D",
  "gene_name": "Interleukin-17D",
  "term_id": "GO:0006954"
}